{
  "term_label": "carbohydrate binding",
  "gene_symbol": "LGALS16",
  "term_id": "GO:0030246",
  "gene_name": "Galectin-16",
  "gene": "UniProtKB:A8MUM7"
}